{
  "gene_name": "Zinc finger protein 844",
  "term_label": "RNA polymerase II transcription regulatory region sequence-specific DNA binding",
  "gene": "UniProtKB:Q08AG5",
  "term_id": "GO:0000977",
  "gene_symbol": "ZNF844"
}